{
  "term_id": "GO:0042776",
  "gene_symbol": "ATP5MF",
  "gene": "UniProtKB:P56134",
  "gene_name": "ATP synthase subunit f, mitochondrial",
  "term_label": "proton motive force-driven mitochondrial ATP synthesis"
}